{
  "gene_name": "1-phosphatidylinositol 4,5-bisphosphate phosphodiesterase epsilon-1",
  "gene": "UniProtKB:Q9P212",
  "term_id": "GO:0046488",
  "term_label": "phosphatidylinositol metabolic process",
  "gene_symbol": "PLCE1"
}